{
  "term_label": "olfactory receptor activity",
  "gene_symbol": "OR5K1",
  "term_id": "GO:0004984",
  "gene_name": "Olfactory receptor 5K1",
  "gene": "UniProtKB:Q8NHB7"
}